{
  "gene": "UniProtKB:Q9NZL3",
  "gene_name": "Zinc finger protein 224",
  "gene_symbol": "ZNF224",
  "term_label": "nucleus",
  "term_id": "GO:0005634"
}